{
  "term_id": "UNKNOWN:0001",
  "term_label": "Unknown molecular function",
  "gene": "UniProtKB:Q7RTS9",
  "gene_name": "Dymeclin",
  "gene_symbol": "DYM"
}